{
  "gene": "UniProtKB:O15467",
  "term_id": "GO:0030335",
  "term_label": "positive regulation of cell migration",
  "gene_symbol": "CCL16",
  "gene_name": "C-C motif chemokine 16"
}